{
  "gene_symbol": "ATF7IP2",
  "gene": "UniProtKB:Q5U623",
  "term_label": "transcription regulator complex",
  "gene_name": "Activating transcription factor 7-interacting protein 2",
  "term_id": "GO:0005667"
}